{
  "gene": "UniProtKB:P20073",
  "term_label": "cytoplasm",
  "term_id": "GO:0005737",
  "gene_symbol": "ANXA7",
  "gene_name": "Annexin A7"
}